{
  "term_id": "GO:0002009",
  "gene_name": "Dystroglycan 1",
  "term_label": "morphogenesis of an epithelium",
  "gene": "UniProtKB:Q14118",
  "gene_symbol": "DAG1"
}